{
  "gene_name": "Gametogenetin-binding protein 2",
  "gene": "UniProtKB:Q9H3C7",
  "term_id": "UNKNOWN:0002",
  "gene_symbol": "GGNBP2",
  "term_label": "Unknown biological process"
}